{
  "gene": "UniProtKB:Q9NZU1",
  "term_id": "GO:0005615",
  "term_label": "extracellular space",
  "gene_symbol": "FLRT1",
  "gene_name": "Leucine-rich repeat transmembrane protein FLRT1"
}